{
  "gene_symbol": "KIAA0930",
  "gene_name": "Uncharacterized protein KIAA0930",
  "gene": "UniProtKB:Q6ICG6",
  "term_id": "UNKNOWN:0002",
  "term_label": "Unknown biological process"
}